heme B transmembrane transporter activity [GO:0170003] (molecular function) References: PMID:15369674, PMID:20610401, PMID:32121449, PMID:9657107 Relationships: is a type of heme transmembrane transporter activity [GO:0015232] Definition: Enables the transfer of heme B from one side of a membrane to the other.